{
  "gene_symbol": "H2BC3",
  "gene_name": "Histone H2B type 1-B",
  "term_label": "structural constituent of chromatin",
  "term_id": "GO:0030527",
  "gene": "UniProtKB:P33778"
}